gap junction channel activity [GO:0005243] (molecular function) Sources: GOC:dgh, GOC:mtg_transport, ISBN:0815340729 Definition: A wide pore channel activity that enables a direct cytoplasmic connection from one cell to an adjacent cell. The gap junction can pass large solutes as well as electrical signals between cells. Gap junctions consist of two gap junction hemi-channels, or connexons, one contributed by each membrane through which the gap junction passes. Relationships: is a type of wide pore channel activity [GO:0022829] Also known as: intercellular channel, innexin channel activity, innexin, connexin Subtypes: gap junction channel activity involved in cell communication by electrical coupling [GO:1903763]